{
  "gene_name": "Ly6_PLAUR domain-containing protein 4",
  "term_label": "Unknown biological process",
  "gene_symbol": "LYPD4",
  "term_id": "UNKNOWN:0002",
  "gene": "UniProtKB:Q6UWN0"
}